{
  "term_label": "cytoplasm",
  "gene_name": "EEF1A lysine methyltransferase 2",
  "term_id": "GO:0005737",
  "gene_symbol": "EEF1AKMT2",
  "gene": "UniProtKB:Q5JPI9"
}